viral capsid, decoration [GO:0098021] (cellular component) Definition: Component of the virus capsid (head), located on the outer head surface. Involved in the stabilization of the head structure and usually non-essential. Subtypes: viral capsid, turret [GO:0039670], viral capsid, fiber [GO:0098022] Sources: GOC:bm, VZ:4398 Also known as: decoration protein Relationships: is a type of virion component [GO:0044423]; is part of viral capsid [GO:0019028]